{
  "gene": "UniProtKB:Q86SG3",
  "term_label": "cytoplasm",
  "gene_symbol": "DAZ4",
  "term_id": "GO:0005737",
  "gene_name": "Deleted in azoospermia protein 4"
}